molybdopterin cofactor metabolic process [GO:0043545] (biological process) Sources: ISSN:09498257 Definition: The chemical reactions and pathways involving the molybdopterin cofactor (Moco), essential for the catalytic activity of some enzymes, e.g. sulfite oxidase, xanthine dehydrogenase, and aldehyde oxidase. The cofactor consists of a mononuclear molybdenum (Mo-molybdopterin) or tungsten ion (W-molybdopterin) coordinated by one or two molybdopterin ligands. Relationships: is a type of phosphate-containing compound metabolic process [GO:0006796]; is_a organophosphate metabolic process [GO:0019637]; is a type of prosthetic group metabolic process [GO:0051189] Also known as: Moco metabolic process, Moco metabolism, molybdopterin cofactor metabolism Subtypes: Mo-molybdopterin cofactor metabolic process [GO:0019720], molybdopterin cofactor biosynthetic process [GO:0032324], molybdopterin cofactor catabolic process [GO:0032325]